{
  "gene_symbol": "BLACAT1",
  "gene_name": "BLACAT1 overlapping LEMD1 locus",
  "gene": "UniProtKB:A0A494BZU2",
  "term_label": "Unknown cellular component",
  "term_id": "UNKNOWN:0003"
}